enzyme activator complex [GO:0150005] (cellular component) Definition: A protein complex capable of activating an enzyme. Activating subunits may dissociate from the catalytic unit before the enzyme is active. References: PMID:16244137, PMID:28710280 Sources: GOC:bhm Relationships: is a type of protein-containing complex [GO:0032991] Subtypes: DNA polymerase processivity factor complex [GO:0044796], DNA recombinase auxiliary factor complex [GO:0120231], GO:0150006, GTPase activator complex [GO:1902773]